response to glucocorticoid [GO:0051384] (biological process) Also known as: response to glucocorticoid stimulus Subtypes: response to corticosterone [GO:0051412], response to cortisone [GO:0051413], response to cortisol [GO:0051414], GO:0051468, GO:0071385, response to dexamethasone [GO:0071548] Relationships: is a type of response to corticosteroid [GO:0031960] References: PMID:9884123 Sources: GOC:ai Definition: Any process that results in a change in state or activity of a cell or an organism (in terms of movement, secretion, enzyme production, gene expression, etc.) as a result of a glucocorticoid stimulus. Glucocorticoids are hormonal C21 corticosteroids synthesized from cholesterol with the ability to bind with the cortisol receptor and trigger similar effects. Glucocorticoids act primarily on carbohydrate and protein metabolism, and have anti-inflammatory effects.